DNA-3-methylguanine glycosylase activity [GO:0052822] (molecular function) Definition: Catalysis of the reaction: DNA containing 3-methylguanine + H2O = DNA with abasic site + 3-methylguanine. This reaction is the hydrolysis of DNA by cleavage of the N-C1' glycosidic bond between the damaged DNA 3-methylguanine and the deoxyribose sugar to remove the 3-methylguanine, leaving an abasic site. References: PMID:10872450, PMID:9224623 Sources: GOC:elh Relationships: is a type of DNA-3-methylbase glycosylase activity [GO:0043733]